{
  "gene": "UniProtKB:O75820",
  "gene_symbol": "ZNF189",
  "gene_name": "Zinc finger protein 189",
  "term_label": "DNA-binding transcription factor activity, RNA polymerase II-specific",
  "term_id": "GO:0000981"
}